{
  "gene_name": "Extended synaptotagmin-2",
  "term_label": "phosphatidylethanolamine binding",
  "term_id": "GO:0008429",
  "gene_symbol": "ESYT2",
  "gene": "UniProtKB:A0FGR8"
}